{
  "gene_name": "GLIPR1-like protein 2",
  "term_id": "GO:0005615",
  "term_label": "extracellular space",
  "gene_symbol": "GLIPR1L2",
  "gene": "UniProtKB:Q4G1C9"
}